{
  "term_id": "GO:0006409",
  "gene_name": "Nucleolar protein 6",
  "gene_symbol": "NOL6",
  "term_label": "tRNA export from nucleus",
  "gene": "UniProtKB:Q9H6R4"
}